{
  "gene_name": "Adipolin",
  "term_id": "GO:0005179",
  "term_label": "hormone activity",
  "gene_symbol": "C1QTNF12",
  "gene": "UniProtKB:Q5T7M4"
}